{
  "term_label": "cell surface",
  "gene_symbol": "ITGA2B",
  "gene": "UniProtKB:P08514",
  "term_id": "GO:0009986",
  "gene_name": "Integrin alpha-IIb"
}